positive regulation of SREBP signaling pathway [GO:2000640] (biological process) Definition: Any process that activates or increases the frequency, rate or extent of the SREBP signaling pathway. Sources: GOC:BHF Also known as: positive regulation of SREBP-mediated signaling pathway, positive regulation of SREBP-mediated signalling pathway Relationships: is_a positive regulation of intracellular signal transduction [GO:1902533]; is a type of regulation of SREBP signaling pathway [GO:2000638]; positively regulates SREBP signaling pathway [GO:0032933] Subtypes: positive regulation of SREBP signaling pathway in response to decreased oxygen levels [GO:0038176]